aliphatic nitrilase activity [GO:0018762] (molecular function) Relationships: is a type of GO:0000257 Also known as: aliphatic nitrile aminohydrolase activity Sources: EC:3.5.5.7 Definition: Catalysis of the reaction: R-CN + H2O = R-COOH + NH3.